{
  "term_id": "GO:0030974",
  "gene": "UniProtKB:Q53GD3",
  "term_label": "thiamine pyrophosphate transmembrane transport",
  "gene_symbol": "SLC44A4",
  "gene_name": "Choline transporter-like protein 4"
}